{
  "gene_name": "Alanyl-tRNA editing protein Aarsd1",
  "gene_symbol": "AARSD1",
  "term_id": "GO:0006450",
  "term_label": "regulation of translational fidelity",
  "gene": "UniProtKB:Q9BTE6"
}